{
  "gene_symbol": "FOXM1",
  "term_label": "DNA-binding transcription factor activity",
  "gene": "UniProtKB:Q08050",
  "gene_name": "Forkhead box protein M1",
  "term_id": "GO:0003700"
}